PRC1 complex [GO:0035102] (cellular component) Also known as: Polycomb repressive complex 1 References: PMID:10412979 Sources: GOC:bf Relationships: is a type of nuclear ubiquitin ligase complex [GO:0000152]; is a type of PcG protein complex [GO:0031519] Note: In Drosophila the core subunits are Pc (Polycomb), Psc (Posterior sex combs), Ph (Polyhomeotic) and Sce (Sex comb extra). In mammals, which have several orthologs for each of the Drosophila core proteins, a family of distinct PRC1-like complexes seem to exist which contain at least some PcG proteins in mutually exclusive manner. Definition: A multiprotein complex that mediates monoubiquitination of lysine residues of histone H2A (lysine-118 in Drosophila or lysine-119 in mammals). The complex is required for stable long-term maintenance of transcriptionally repressed states and is involved in chromatin remodeling.